{
  "term_id": "GO:0044331",
  "gene": "UniProtKB:P55285",
  "gene_symbol": "CDH6",
  "term_label": "cell-cell adhesion mediated by cadherin",
  "gene_name": "Cadherin-6"
}